{
  "term_label": "structural constituent of cytoskeleton",
  "gene": "UniProtKB:O15144",
  "gene_symbol": "ARPC2",
  "gene_name": "Actin-related protein 2_3 complex subunit 2",
  "term_id": "GO:0005200"
}